{
  "gene_symbol": "SERPINB9",
  "gene_name": "Serpin B9",
  "term_id": "UNKNOWN:0002",
  "term_label": "Unknown biological process",
  "gene": "UniProtKB:P50453"
}